{
  "term_label": "mRNA splicing, via spliceosome",
  "gene_symbol": "RBMY1F",
  "gene": "UniProtKB:Q15415",
  "term_id": "GO:0000398",
  "gene_name": "RNA-binding motif protein, Y chromosome, family 1 member F_J"
}